{
  "term_id": "GO:0086011",
  "term_label": "membrane repolarization during action potential",
  "gene_symbol": "KCNE4",
  "gene": "UniProtKB:Q8WWG9",
  "gene_name": "Potassium voltage-gated channel subfamily E member 4"
}